{
  "gene": "UniProtKB:P48764",
  "term_label": "sodium:proton antiporter activity",
  "gene_name": "Sodium_hydrogen exchanger 3",
  "gene_symbol": "SLC9A3",
  "term_id": "GO:0015385"
}